{
  "gene_symbol": "HSD3B1",
  "gene_name": "3 beta-hydroxysteroid dehydrogenase_Delta 5--4-isomerase type 1",
  "term_id": "GO:0005737",
  "term_label": "cytoplasm",
  "gene": "UniProtKB:P14060"
}